{
  "term_id": "GO:0005737",
  "gene_symbol": "PPP4C",
  "gene": "UniProtKB:P60510",
  "gene_name": "Serine_threonine-protein phosphatase 4 catalytic subunit",
  "term_label": "cytoplasm"
}